{
  "gene_name": "Guanylyl cyclase-activating protein 1",
  "term_id": "GO:0008048",
  "gene_symbol": "GUCA1A",
  "term_label": "calcium sensitive guanylate cyclase activator activity",
  "gene": "UniProtKB:P43080"
}